imaginal disc-derived female genitalia development [GO:0007486] (BP) Definition: The process whose specific outcome is the progression of the female genitalia over time, from formation as part of the genital disc to the mature structure. An example of this is found in Drosophila melanogaster. Also known as: female genital development Sources: GOC:ai, GOC:sensu Relationships: is a type of imaginal disc-derived genitalia development [GO:0007484]; is a type of female genitalia development [GO:0030540]